{
  "gene_symbol": "TRBV24-1",
  "gene": "UniProtKB:A0A075B6N3",
  "term_id": "GO:0005886",
  "gene_name": "T cell receptor beta variable 24-1",
  "term_label": "plasma membrane"
}